{
  "gene_name": "Dynein axonemal assembly factor 1",
  "term_id": "GO:0070840",
  "gene_symbol": "DNAAF1",
  "gene": "UniProtKB:Q8NEP3",
  "term_label": "dynein complex binding"
}